{
  "gene": "UniProtKB:O95415",
  "term_id": "UNKNOWN:0001",
  "gene_name": "Membrane protein BRI3",
  "term_label": "Unknown molecular function",
  "gene_symbol": "BRI3"
}